iron acquisition from host [GO:0044847] (biological process) Also known as: iron acquisition, iron acquisition by symbiont from host, acquisition by symbiont of nutrients from host via siderophores, iron acquisition by symbiont from host heme, acquisition by organism of nutrients from host via siderophores, heme acquisition Relationships: is a type of acquisition of nutrients from host [GO:0044002] References: PMID:15487950, PMID:22865843 Definition: The process by which a symbiont acquires iron from its host, either from heme or other iron containing molecules such as transferrin and lactoferrin. Begins with either the secretion of symbiont gene products that bind iron- or heme-containing molecules (siderophores and hemophores) from the symbiont cell into the host, or by expression of receptors that bind iron- or heme-containing molecules on the symbiont cell surface. Ends when the iron-containing compound is transported into the symbiont cell.